{
  "gene_symbol": "OR13C9",
  "term_id": "GO:0005886",
  "gene": "UniProtKB:Q8NGT0",
  "term_label": "plasma membrane",
  "gene_name": "Olfactory receptor 13C9"
}